{
  "gene": "UniProtKB:O15228",
  "term_id": "GO:0005778",
  "gene_name": "Dihydroxyacetone phosphate acyltransferase",
  "gene_symbol": "GNPAT",
  "term_label": "peroxisomal membrane"
}